{
  "gene_symbol": "GABRB3",
  "term_label": "GABA-A receptor complex",
  "gene": "UniProtKB:P28472",
  "gene_name": "Gamma-aminobutyric acid receptor subunit beta-3",
  "term_id": "GO:1902711"
}